transcription corepressor binding [GO:0001222] (molecular function) Sources: GOC:krc Relationships: is a type of transcription coregulator binding [GO:0001221] Also known as: RNA polymerase II transcription corepressor binding Definition: Binding to a transcription corepressor, a protein involved in negative regulation of transcription via protein-protein interactions with transcription factors and other proteins that negatively regulate transcription. Transcription corepressors do not bind DNA directly, but rather mediate protein-protein interactions between repressing transcription factors and the basal transcription machinery.